small ribosomal subunit processing complex [GO:0140638] (cellular component) Also known as: small ribosomal subunit maturation complex References: PMID:21849504, PMID:25064857 Sources: GOC:lnp Definition: A small heterodimeric protein complex that is required during early maturation of nascent 40S ribosomal subunits. The complex has endonuclease activity, it interacts with the small ribosomal subunit pre-rRNA and cleave it it to produce the mature 18S (or small ribosomal subunit) rRNA. In S. cerevisiae it is composed of Rcl1p and Bms1p. Relationships: is a type of endoribonuclease complex [GO:1902555]